2-methylisocitrate dehydratase activity [GO:0047456] (molecular function) Relationships: is_a hydro-lyase activity [GO:0016836] Also known as: (2S,3R)-3-hydroxybutane-1,2,3-tricarboxylate hydro-lyase [(Z)-but-2-ene-1,2,3-tricarboxylate-forming], (2S,3R)-3-hydroxybutane-1,2,3-tricarboxylate hydro-lyase activity Sources: EC:4.2.1.99, RHEA:17941 Definition: Catalysis of the reaction: (2S,3R)-3-hydroxybutane-1,2,3-tricarboxylate = cis-2-methylaconitate + H2O.